(R)-carnitine transmembrane transport [GO:1902270] (biological process) Definition: The process in which (R)-carnitine is transported across a membrane. Regulation: RO_0002211 by regulation of (R)-carnitine transmembrane transport [GO:1902272]; negatively regulated by GO:1902273; positively regulated by positive regulation of (R)-carnitine transmembrane transport [GO:1902274] References: PMID:23755272 Sources: GOC:TermGenie Relationships: is a type of GO:1900749; is a type of carnitine transmembrane transport [GO:1902603]